{
  "gene_name": "Immunoglobulin kappa joining 2 (Fragment)",
  "gene": "UniProtKB:A0A0A0MT85",
  "term_id": "UNKNOWN:0001",
  "gene_symbol": "IGKJ2",
  "term_label": "Unknown molecular function"
}